{
  "term_id": "UNKNOWN:0002",
  "gene_symbol": "C11orf52",
  "gene_name": "Uncharacterized protein C11orf52",
  "gene": "UniProtKB:Q96A22",
  "term_label": "Unknown biological process"
}